positive regulation of methane biosynthetic process from methylamine [GO:1900350] (biological process) Definition: Any process that activates or increases the frequency, rate or extent of methane biosynthetic process from methylamine. Sources: GOC:TermGenie, GOC:mengo_curators Also known as: up regulation of methane biosynthetic process from methylamine, up-regulation of methane biosynthetic process from methylamine, upregulation of methane biosynthetic process from methylamine, activation of methane biosynthetic process from methylamine Relationships: is a type of GO:0033240; is a type of regulation of methane biosynthetic process from methylamine [GO:1900348]; is a type of positive regulation of alkane biosynthetic process [GO:1901579]; is a type of positive regulation of cellular respiration [GO:1901857]; RO_0002213 methane biosynthetic process from methylamine [GO:2001128]